glucuronoarabinoxylan endo-1,4-beta-xylanase activity [GO:0033940] (MF) Definition: Catalysis of the endohydrolysis of (1->4)-beta-D-xylosyl links in some glucuronoarabinoxylans. Relationships: is a type of xylanase activity [GO:0097599] Also known as: endoarabinoxylanase activity, feraxan endoxylanase activity, feraxanase activity, glucuronoarabinoxylan 1,4-beta-D-xylanohydrolase activity, glucuronoxylan xylanohydrolase activity, glucuronoxylan xylohydrolase activity, glucuronoxylanase activity Sources: EC:3.2.1.136